central nervous system myelin maintenance [GO:0032286] (biological process) Definition: The process in which the structure and material content of mature central nervous system myelin is kept in a functional state. Sources: GOC:dgh Also known as: central nervous system myelin sheath maintenance, myelin maintenance in central nervous system Relationships: is a type of myelin maintenance [GO:0043217]; is part of GO:0022010